{
  "term_label": "regulation of insulin-like growth factor receptor signaling pathway",
  "gene": "UniProtKB:P17936",
  "term_id": "GO:0043567",
  "gene_symbol": "IGFBP3",
  "gene_name": "Insulin-like growth factor-binding protein 3"
}